eye morphogenesis [GO:0048592] (biological process) Relationships: is_a sensory organ morphogenesis [GO:0090596]; is part of eye development [GO:0001654] Definition: The process in which the anatomical structures of the eye are generated and organized. Subtypes: GO:0001745, Bolwig's organ morphogenesis [GO:0001746], GO:0048048, post-embryonic eye morphogenesis [GO:0048050], GO:0048593 Sources: GOC:jid, GOC:mtg_sensu